{
  "term_label": "axon",
  "gene_symbol": "MYOT",
  "gene_name": "Myotilin",
  "term_id": "GO:0030424",
  "gene": "UniProtKB:Q9UBF9"
}